{
  "gene_name": "C-terminal-binding protein 1",
  "term_id": "GO:0006357",
  "gene": "UniProtKB:Q13363",
  "term_label": "regulation of transcription by RNA polymerase II",
  "gene_symbol": "CTBP1"
}